{
  "term_id": "UNKNOWN:0001",
  "gene_symbol": "CLRN2",
  "term_label": "Unknown molecular function",
  "gene": "UniProtKB:A0PK11",
  "gene_name": "Clarin-2"
}